{
  "term_id": "GO:0005978",
  "gene_symbol": "GYS1",
  "gene": "UniProtKB:P13807",
  "term_label": "glycogen biosynthetic process",
  "gene_name": "Glycogen [starch] synthase, muscle"
}